{
  "gene": "UniProtKB:Q9H361",
  "term_label": "ribonucleoprotein complex",
  "term_id": "GO:1990904",
  "gene_name": "Polyadenylate-binding protein 3",
  "gene_symbol": "PABPC3"
}